{
  "term_label": "Unknown cellular component",
  "gene": "UniProtKB:A0A0B4J1X5",
  "term_id": "UNKNOWN:0003",
  "gene_symbol": "IGHV3-74",
  "gene_name": "Immunoglobulin heavy variable 3-74"
}